{
  "term_label": "protein retention in ER lumen",
  "gene_symbol": "KDELR1",
  "gene_name": "ER lumen protein-retaining receptor 1",
  "term_id": "GO:0006621",
  "gene": "UniProtKB:P24390"
}